{
  "gene_symbol": "H2BC17",
  "term_label": "nucleus",
  "term_id": "GO:0005634",
  "gene_name": "Histone H2B type 1-O",
  "gene": "UniProtKB:P23527"
}